AUA codon-amino acid adaptor activity [GO:0033435] (molecular function) Also known as: ATA codon-amino acid adaptor activity, isoleucine tRNA Note: Note that in the standard genetic code, ATA codes for isoleucine. Relationships: is a type of GO:0030533 Sources: GOC:mah Definition: A triplet codon-amino acid adaptor activity that recognizes an AUA codon.